{
  "gene": "UniProtKB:Q9NZU7",
  "gene_symbol": "CABP1",
  "gene_name": "Calcium-binding protein 1",
  "term_id": "GO:0007602",
  "term_label": "phototransduction"
}